{
  "term_label": "neuron projection development",
  "term_id": "GO:0031175",
  "gene_symbol": "DTNBP1",
  "gene_name": "Dysbindin",
  "gene": "UniProtKB:Q96EV8"
}